lung development [GO:0030324] (biological process) Definition: The process whose specific outcome is the progression of the lung over time, from its formation to the mature structure. In all air-breathing vertebrates the lungs are developed from the ventral wall of the oesophagus as a pouch which divides into two sacs. In amphibians and many reptiles the lungs retain very nearly this primitive sac-like character, but in the higher forms the connection with the esophagus becomes elongated into the windpipe and the inner walls of the sacs become more and more divided, until, in the mammals, the air spaces become minutely divided into tubes ending in small air cells, in the walls of which the blood circulates in a fine network of capillaries. In mammals the lungs are more or less divided into lobes, and each lung occupies a separate cavity in the thorax. Relationships: is a type of animal organ development [GO:0048513]; is part of respiratory tube development [GO:0030323]; is part of respiratory system development [GO:0060541] Sources: GOC:jid, UBERON:0002048 Subtypes: right lung development [GO:0060458], left lung development [GO:0060459]